DNA replication, synthesis of primer [GO:0006269] (BP) Also known as: DNA priming, DNA replication, synthesis of DNA primer, DNA replication, synthesis of RNA primer, replication priming Relationships: is a type of RNA biosynthetic process [GO:0032774]; is part of GO:0006261 References: PMID:11395402, PMID:38203225, PMID:38492718 Definition: The synthesis of a short nucleotide polymer using one strand of unwound DNA as a template. The product is usually a RNA molecule between 4-15 nucleotides long that provides a free 3'-OH that can be extended by DNA-directed DNA polymerases. In certain conditions, for example in response to DNA damage, some primases synthesize a DNA primer.